{
  "gene_name": "Putative Ras-related protein Rab-1C",
  "term_id": "GO:0000045",
  "term_label": "autophagosome assembly",
  "gene": "UniProtKB:Q92928",
  "gene_symbol": "RAB1C"
}